{
  "gene": "UniProtKB:Q9GZZ6",
  "gene_symbol": "CHRNA10",
  "term_id": "GO:0034220",
  "gene_name": "Neuronal acetylcholine receptor subunit alpha-10",
  "term_label": "monoatomic ion transmembrane transport"
}